negative regulation of maltotriulose transport [GO:1900325] (biological process) Sources: GOC:TermGenie, GOC:mengo_curators Also known as: down regulation of maltotriulose transport, down-regulation of maltotriulose transport, downregulation of maltotriulose transport, inhibition of maltotriulose transport Relationships: is a type of GO:0051051; is a type of regulation of maltotriulose transport [GO:1900324]; negatively regulates maltotriulose transport [GO:2001090] Definition: Any process that stops, prevents or reduces the frequency, rate or extent of maltotriulose transport.